positive regulation of sprouting of injured axon [GO:0048687] (biological process) Definition: Any process that activates, maintains or increases the rate of sprouting of an injured axon. Sources: GOC:dgh, GOC:dph, GOC:jid, GOC:lm Also known as: up regulation of sprouting of injured axon, up-regulation of sprouting of injured axon, upregulation of sprouting of injured axon, activation of sprouting of injured axon, stimulation of sprouting of injured axon Subtypes: GO:0048691, positive regulation of collateral sprouting of injured axon [GO:0048694], positive regulation of formation of growth cone in injured axon [GO:1905944] Relationships: is a type of positive regulation of cell growth [GO:0030307]; is a type of positive regulation of developmental growth [GO:0048639]; is a type of positive regulation of axon regeneration [GO:0048680]; is a type of GO:0048686; positively regulates sprouting of injured axon [GO:0048682]